oxidoreductase activity, acting on the aldehyde or oxo group of donors, oxygen as acceptor [GO:0016623] (molecular function) Subtypes: GO:0004031, 4-hydroxyphenylpyruvate oxidase activity [GO:0018490], glyoxal oxidase activity [GO:0046569], pyruvate oxidase activity [GO:0047112], GO:0047969, oxalate oxidase activity [GO:0050162], pyruvate oxidase (CoA-acetylating) activity [GO:0050244] Relationships: is a type of oxidoreductase activity, acting on the aldehyde or oxo group of donors [GO:0016903] Definition: Catalysis of an oxidation-reduction (redox) reaction in which an aldehyde or ketone (oxo) group acts as a hydrogen or electron donor and reduces oxygen. Sources: EC:1.2.3.-